detoxification of iron ion [GO:1990461] (biological process) Definition: Any process that reduces or removes the toxicity of iron ion. These include transport of iron away from sensitive areas and to compartments or complexes whose purpose is sequestration of iron ion. Relationships: is a type of detoxification of inorganic compound [GO:0061687]; is part of response to iron ion [GO:0010039] References: PMID:23064556 Sources: GOC:sart